{
  "term_label": "Unknown biological process",
  "term_id": "UNKNOWN:0002",
  "gene": "UniProtKB:Q9BVG9",
  "gene_symbol": "PTDSS2",
  "gene_name": "Phosphatidylserine synthase 2"
}